{
  "gene": "UniProtKB:Q8NDZ4",
  "gene_symbol": "DIPK2A",
  "term_id": "UNKNOWN:0001",
  "term_label": "Unknown molecular function",
  "gene_name": "Divergent protein kinase domain 2A"
}